{
  "gene": "UniProtKB:P21291",
  "term_label": "actinin binding",
  "gene_name": "Cysteine and glycine-rich protein 1",
  "gene_symbol": "CSRP1",
  "term_id": "GO:0042805"
}